{
  "gene": "UniProtKB:Q6XYB7",
  "gene_symbol": "LBX2",
  "gene_name": "Transcription factor LBX2",
  "term_label": "regulation of transcription by RNA polymerase II",
  "term_id": "GO:0006357"
}